{
  "term_label": "Unknown cellular component",
  "gene_name": "T cell receptor alpha joining 22 (Fragment)",
  "term_id": "UNKNOWN:0003",
  "gene": "UniProtKB:A0A075B6Z0",
  "gene_symbol": "TRAJ22"
}